{
  "gene_symbol": "AGRN",
  "gene": "UniProtKB:O00468",
  "term_id": "GO:0007268",
  "gene_name": "Agrin",
  "term_label": "chemical synaptic transmission"
}